{
  "gene_name": "Ubiquitin carboxyl-terminal hydrolase 17-like protein 5",
  "term_label": "regulation of apoptotic process",
  "term_id": "GO:0042981",
  "gene_symbol": "USP17L5",
  "gene": "UniProtKB:A8MUK1"
}